{
  "gene_symbol": "SHARPIN",
  "term_label": "LUBAC complex",
  "term_id": "GO:0071797",
  "gene": "UniProtKB:Q9H0F6",
  "gene_name": "Sharpin"
}